{
  "term_id": "GO:0039706",
  "gene_symbol": "DKK2",
  "term_label": "co-receptor binding",
  "gene": "UniProtKB:Q9UBU2",
  "gene_name": "Dickkopf-related protein 2"
}